{
  "gene_name": "Potassium voltage-gated channel subfamily D member 1",
  "gene_symbol": "KCND1",
  "term_id": "GO:0043197",
  "term_label": "dendritic spine",
  "gene": "UniProtKB:Q9NSA2"
}